positive regulation of nitric oxide biosynthetic process [GO:0045429] (BP) Sources: GOC:go_curators Also known as: positive regulation of nitric oxide anabolism, positive regulation of nitric oxide biosynthesis, positive regulation of nitric oxide formation, positive regulation of nitric oxide synthesis, up regulation of nitric oxide biosynthetic process, up-regulation of nitric oxide biosynthetic process, upregulation of nitric oxide biosynthetic process, activation of nitric oxide biosynthetic process, stimulation of nitric oxide biosynthetic process Definition: Any process that activates or increases the frequency, rate or extent of the chemical reactions and pathways resulting in the formation of nitric oxide. Relationships: is a type of positive regulation of biosynthetic process [GO:0009891]; is a type of regulation of nitric oxide biosynthetic process [GO:0045428]; positively regulates nitric oxide biosynthetic process [GO:0006809]